{
  "gene": "UniProtKB:O60264",
  "term_id": "GO:0003682",
  "term_label": "chromatin binding",
  "gene_symbol": "SMARCA5",
  "gene_name": "SWI_SNF-related matrix-associated actin-dependent regulator of chromatin subfamily A member 5"
}